5-pyridoxate dioxygenase activity [GO:0047592] (molecular function) Definition: Catalysis of the reaction: 5-pyridoxate + NADPH + O2 = 2-(acetamidomethylene)-3-(hydroxymethyl)succinate) + NADP+. Also known as: 5-pyridoxate oxidase activity Sources: RHEA:11152 Relationships: is a type of oxidoreductase activity, acting on paired donors, with incorporation or reduction of molecular oxygen, NAD(P)H as one donor, and incorporation of one atom of oxygen [GO:0016709]